{
  "gene_symbol": "TEX15",
  "term_id": "UNKNOWN:0001",
  "term_label": "Unknown molecular function",
  "gene": "UniProtKB:Q9BXT5",
  "gene_name": "Testis-expressed protein 15"
}